{
  "gene_name": "Somatomedin-B and thrombospondin type-1 domain-containing protein",
  "term_id": "UNKNOWN:0003",
  "term_label": "Unknown cellular component",
  "gene_symbol": "SBSPON",
  "gene": "UniProtKB:Q8IVN8"
}